surfactant secretion [GO:0160069] (biological process) Relationships: is a type of secretion [GO:0046903]; is part of surfactant homeostasis [GO:0043129] References: PMID:19824815 Definition: The regulated release of surfactant by a cell or tissue.